glutathione transmembrane import into vacuole [GO:0071996] (biological process) Definition: The directed movement of glutathione into the vacuole across the vacuolar membrane. Sources: GOC:mah Relationships: is_a vacuolar transmembrane transport [GO:0034486]; is a type of glutathione transmembrane transport [GO:0034775] Also known as: glutathione transport into vacuole